guanosine deaminase activity [GO:0047974] (molecular function) Sources: EC:3.5.4.15, MetaCyc:GUANOSINE-DEAMINASE-RXN Also known as: guanosine aminase activity, guanosine aminohydrolase activity Relationships: is a type of hydrolase activity, acting on carbon-nitrogen (but not peptide) bonds, in cyclic amidines [GO:0016814]; is a type of GO:0019239 Definition: Catalysis of the reaction: guanosine + H2O = xanthosine + NH3.